D-dopachrome decarboxylase activity [GO:0033981] (molecular function) Sources: EC:4.1.1.84, RHEA:18441 Relationships: is a type of carboxy-lyase activity [GO:0016831] Definition: Catalysis of the reaction: D-dopachrome + H+ = 5,6-dihydroxyindole + CO2. Also known as: dopachrome conversion activity, dopachrome decarboxylase activity, D-dopachrome carboxy-lyase (5,6-dihydroxyindole-forming) activity, D-dopachrome carboxy-lyase activity, D-dopachrome tautomerase activity, D-tautomerase activity, phenylpyruvate tautomerase II activity